GGU codon-amino acid adaptor activity [GO:0033461] (molecular function) Definition: A triplet codon-amino acid adaptor activity that recognizes a GGU codon. Sources: GOC:mah Also known as: GGT codon-amino acid adaptor activity, glycine tRNA Note: Note that in the standard genetic code, GGT codes for glycine. Relationships: is_a GO:0030533